{
  "gene": "UniProtKB:P36575",
  "term_id": "GO:0001664",
  "term_label": "G protein-coupled receptor binding",
  "gene_name": "Arrestin-C",
  "gene_symbol": "ARR3"
}